regulation of vacuole organization [GO:0044088] (biological process) Relationships: is_a regulation of organelle organization [GO:0033043]; regulates vacuole organization [GO:0007033] Subtypes: regulation of vacuole fusion, non-autophagic [GO:0032889], positive regulation of vacuole organization [GO:0044090], GO:1905671, GO:2000785 Definition: Any process that modulates the frequency, rate or extent of a process involved in the formation, arrangement of constituent parts, or disassembly of a vacuole. Sources: GOC:jl, GOC:mah Also known as: regulation of vacuole organisation, regulation of vacuole biogenesis